{
  "gene": "UniProtKB:Q5T7V8",
  "gene_name": "RAB6-interacting golgin",
  "term_id": "UNKNOWN:0001",
  "term_label": "Unknown molecular function",
  "gene_symbol": "GORAB"
}